{
  "term_label": "G protein-coupled receptor signaling pathway, coupled to cyclic nucleotide second messenger",
  "gene_symbol": "CHRM1",
  "gene_name": "Muscarinic acetylcholine receptor M1",
  "term_id": "GO:0007187",
  "gene": "UniProtKB:P11229"
}